{
  "term_id": "GO:0000828",
  "gene_name": "Inositol-trisphosphate 3-kinase C",
  "gene_symbol": "ITPKC",
  "term_label": "inositol hexakisphosphate kinase activity",
  "gene": "UniProtKB:Q96DU7"
}